{
  "term_id": "UNKNOWN:0002",
  "gene": "UniProtKB:Q6Q0C1",
  "term_label": "Unknown biological process",
  "gene_symbol": "SLC25A47",
  "gene_name": "Solute carrier family 25 member 47"
}